structural constituent of nuclear lamina [GO:0160123] (molecular function) Relationships: is a type of structural molecule activity [GO:0005198] Definition: The action of a molecule that contributes to the structural integrity of nuclear lamina. References: PMID:2824113, PMID:31434876